{
  "term_id": "GO:0005634",
  "term_label": "nucleus",
  "gene_symbol": "ELF2",
  "gene": "UniProtKB:Q15723",
  "gene_name": "ETS-related transcription factor Elf-2"
}